{
  "term_id": "GO:0055078",
  "gene": "UniProtKB:P55017",
  "gene_name": "Solute carrier family 12 member 3",
  "term_label": "sodium ion homeostasis",
  "gene_symbol": "SLC12A3"
}